{
  "gene_symbol": "SF3A1",
  "gene": "UniProtKB:Q15459",
  "gene_name": "Splicing factor 3A subunit 1",
  "term_id": "GO:0005686",
  "term_label": "U2 snRNP"
}